negative regulation of muscle hypertrophy [GO:0014741] (biological process) Relationships: is a type of regulation of muscle hypertrophy [GO:0014743]; is a type of GO:0051241; negatively regulates muscle hypertrophy [GO:0014896] Subtypes: negative regulation of cardiac muscle hypertrophy [GO:0010614], negative regulation of skeletal muscle hypertrophy [GO:1904205], negative regulation of smooth muscle hypertrophy [GO:1905148] Sources: GOC:mtg_muscle Definition: Any process that stops, prevents, or reduces the frequency, rate, or extent of muscle hypertrophy.